prephenate(2-) catabolic process [GO:1901746] (biological process) Also known as: prephenate breakdown, prephenate catabolism, prephenate degradation, prephenate(2-) breakdown, prephenate(2-) catabolism, prephenate(2-) degradation References: PMID:16752890 Sources: GOC:TermGenie, GOC:yaf Definition: The chemical reactions and pathways resulting in the breakdown of prephenate(2-). Relationships: is a type of dicarboxylic acid catabolic process [GO:0043649]